{
  "gene_symbol": "NR2F2",
  "term_id": "GO:0007399",
  "gene": "UniProtKB:P24468",
  "gene_name": "COUP transcription factor 2",
  "term_label": "nervous system development"
}